4-hydroxybutyrate dehydrogenase activity [GO:0047577] (molecular function) Sources: EC:1.1.1.61, RHEA:23948 Definition: Catalysis of the reaction: 4-hydroxybutanoate + NAD+ = H+ + NADH + succinate semialdehyde. Also known as: 4-hydroxybutanoate:NAD+ oxidoreductase activity, gamma-hydroxybutyrate dehydrogenase activity Relationships: is a type of GO:0016616